negative regulation of branch elongation involved in ureteric bud branching [GO:0072096] (biological process) Relationships: is_a GO:0048640; is a type of regulation of branch elongation involved in ureteric bud branching [GO:0072095]; negatively regulates branch elongation involved in ureteric bud branching [GO:0060681] Definition: Any process that reduces the frequency, rate or extent of branch elongation involved in ureteric bud branching, the growth of a branch of the ureteric bud along its axis. Sources: GOC:mtg_kidney_jan10